{
  "term_label": "motor neuron axon guidance",
  "gene_symbol": "SEMA3A",
  "gene_name": "Semaphorin-3A",
  "gene": "UniProtKB:Q14563",
  "term_id": "GO:0008045"
}